{
  "gene": "UniProtKB:Q8NGB2",
  "term_id": "UNKNOWN:0002",
  "gene_symbol": "OR4C5",
  "gene_name": "Olfactory receptor 4C5",
  "term_label": "Unknown biological process"
}